{
  "term_id": "GO:0005634",
  "gene_symbol": "SMNDC1",
  "gene": "UniProtKB:O75940",
  "gene_name": "Survival of motor neuron-related-splicing factor 30",
  "term_label": "nucleus"
}